{
  "gene": "UniProtKB:P32314",
  "term_label": "nucleus",
  "gene_name": "Forkhead box protein N2",
  "term_id": "GO:0005634",
  "gene_symbol": "FOXN2"
}